{
  "gene_symbol": "ODF4",
  "term_label": "Unknown molecular function",
  "gene_name": "Outer dense fiber protein 4",
  "term_id": "UNKNOWN:0001",
  "gene": "UniProtKB:Q2M2E3"
}